{
  "gene_name": "Homeobox protein DLX-5",
  "gene_symbol": "DLX5",
  "gene": "UniProtKB:P56178",
  "term_id": "GO:0000978",
  "term_label": "RNA polymerase II cis-regulatory region sequence-specific DNA binding"
}